{
  "term_id": "UNKNOWN:0002",
  "term_label": "Unknown biological process",
  "gene_symbol": "GNE",
  "gene": "UniProtKB:Q9Y223",
  "gene_name": "Bifunctional UDP-N-acetylglucosamine 2-epimerase_N-acetylmannosamine kinase"
}